{
  "term_label": "plasma membrane",
  "gene": "UniProtKB:Q6ZMH5",
  "gene_name": "Zinc transporter ZIP5",
  "gene_symbol": "SLC39A5",
  "term_id": "GO:0005886"
}